{
  "term_label": "acetylcholine receptor binding",
  "gene_name": "Prostate stem cell antigen",
  "gene": "UniProtKB:O43653",
  "term_id": "GO:0033130",
  "gene_symbol": "PSCA"
}